{
  "gene_name": "Alkaline phosphatase, placental type",
  "term_id": "GO:0004035",
  "gene": "UniProtKB:P05187",
  "gene_symbol": "ALPP",
  "term_label": "alkaline phosphatase activity"
}